{
  "gene_symbol": "PPIAL4C",
  "gene": "UniProtKB:A0A0B4J2A2",
  "gene_name": "Peptidyl-prolyl cis-trans isomerase A-like 4C",
  "term_label": "cytoplasm",
  "term_id": "GO:0005737"
}